nuclear outer membrane organization [GO:0071764] (biological process) Definition: A process that is carried out at the cellular level which results in the assembly, arrangement of constituent parts, or disassembly of the nuclear outer membrane. Sources: GOC:mah Also known as: nuclear outer membrane organisation, nuclear outer membrane organization and biogenesis Relationships: is a type of nuclear membrane organization [GO:0071763]